adipokinetic hormone binding [GO:0097004] (MF) Relationships: is a type of GO:0017046 Definition: Binding to an adipokinetic hormone. Adipokinetic hormones (AKHs) are peptide hormones that are involved in the mobilization of sugar and lipids from the insect fat body during energy-requiring activities such as flight and locomotion. They also contribute to hemolymph sugar homeostasis. References: PMID:11904407 Sources: GOC:sart Also known as: AKH binding